{
  "gene_symbol": "BAG3",
  "term_label": "protein-folding chaperone binding",
  "term_id": "GO:0051087",
  "gene_name": "BAG family molecular chaperone regulator 3",
  "gene": "UniProtKB:O95817"
}